cephalosporin-C transaminase activity [GO:0047740] (MF) Also known as: L-alanine:cephalosporin-C aminotransferase activity, cephalosporin C aminotransferase activity, cephalosporin-C:2-oxoglutarate aminotransferase activity Definition: Catalysis of the reaction: (7R)-7-(5-carboxylato-5-oxopentanamido)deacetylcephalosporanate + D-glutamate = 2-oxoglutarate + cephalosporin C. Sources: EC:2.6.1.74, RHEA:14553 Relationships: is_a transaminase activity [GO:0008483]